{
  "term_id": "GO:0070475",
  "gene": "UniProtKB:Q9BRP7",
  "gene_symbol": "FDXACB1",
  "term_label": "rRNA base methylation",
  "gene_name": "Ferredoxin-fold anticodon-binding domain-containing protein 1"
}